{
  "gene_symbol": "PCBP4",
  "gene_name": "Poly(rC)-binding protein 4",
  "term_id": "GO:0006357",
  "gene": "UniProtKB:P57723",
  "term_label": "regulation of transcription by RNA polymerase II"
}